{
  "gene_symbol": "HTRA4",
  "term_label": "Unknown cellular component",
  "gene_name": "Serine protease HTRA4",
  "term_id": "UNKNOWN:0003",
  "gene": "UniProtKB:P83105"
}